{
  "gene_symbol": "LGI2",
  "gene_name": "Leucine-rich repeat LGI family member 2",
  "term_label": "Unknown molecular function",
  "term_id": "UNKNOWN:0001",
  "gene": "UniProtKB:Q8N0V4"
}